{
  "term_id": "UNKNOWN:0003",
  "gene_symbol": "MINDY4B",
  "term_label": "Unknown cellular component",
  "gene": "UniProtKB:A8MYZ0",
  "gene_name": "Inactive ubiquitin carboxyl-terminal hydrolase MINDY-4B"
}